{
  "gene": "UniProtKB:Q5BJD5",
  "gene_name": "Transmembrane protein 41B",
  "term_id": "UNKNOWN:0001",
  "gene_symbol": "TMEM41B",
  "term_label": "Unknown molecular function"
}